ganglioside biosynthetic process [GO:0001574] (BP) References: PMID:35536927 Also known as: ganglio-series glycosphingolipid biosynthesis, ganglioside anabolism, ganglioside biosynthesis, ganglioside formation, ganglioside synthesis Relationships: is a type of ganglioside metabolic process [GO:0001573]; is a type of glycosphingolipid biosynthetic process [GO:0006688]; is a type of ceramide biosynthetic process [GO:0046513] Definition: The chemical reactions and pathways resulting in the formation of gangliosides that begins with the synthesis of a tetrasaccharide core Gal-beta-1,3-GalNAc-beta-1,4-Gal-beta-1,4-Glc-ceramide. This core can be further elongated with the sequential addition of various carbohydrate units including the addition of one or more sialic acid residues.